cerebellar molecular layer structural organization [GO:0021689] (biological process) Relationships: is a type of anatomical structure arrangement [GO:0048532]; is part of cerebellar molecular layer morphogenesis [GO:0021687]; is part of cerebellar cortex structural organization [GO:0021698] Also known as: cerebellar molecular layer structural organisation Sources: GOC:cls, GOC:dgh, GOC:dph, GOC:jid, GO_REF:0000021 Definition: The process that contributes to the act of creating the structural organization of the cerebellar molecular layer. This process pertains to the physical shaping of a rudimentary structure. The molecular layer is the outermost layer of the cerebellar cortex. It contains the parallel fibers of the granule cells, interneurons such as stellate and basket cells, and the dendrites of the underlying Purkinje cells.